regulation of membrane protein ectodomain proteolysis [GO:0051043] (biological process) Definition: Any process that modulates the frequency, rate or extent of the proteolytic cleavage of transmembrane proteins and release of their ectodomain (extracellular domain). Sources: GOC:ai Relationships: is a type of regulation of proteolysis [GO:0030162]; is a type of GO:0042176; regulates GO:0006509 Subtypes: positive regulation of membrane protein ectodomain proteolysis [GO:0051044], negative regulation of membrane protein ectodomain proteolysis [GO:0051045]